protein O-linked glycosylation via N-acetyl-galactosamine [GO:0016266] (biological process) References: PMID:10580130, PMID:35536936 Subtypes: GO:0140264 Also known as: O-glycan processing, core O-glycan biosynthetic process, mucin-type O-glycan synthesis, protein O-linked GalNAcylation Relationships: is a type of protein O-linked glycosylation [GO:0006493] Definition: A glycoprotein biosynthetic process starting with the covalent linkage of an N-acetyl-galactosamine via an alpha-glycosidic bond to the oxygen atom of a serine or threonine side chain in a protein, which can be further elongated with the sequential addition of sugar units resulting in the formation of a protein O-linked glycan.